{
  "gene_name": "N-alpha-acetyltransferase 40",
  "term_label": "Unknown biological process",
  "term_id": "UNKNOWN:0002",
  "gene": "UniProtKB:Q86UY6",
  "gene_symbol": "NAA40"
}